{
  "term_id": "GO:0022625",
  "gene": "UniProtKB:P05386",
  "gene_name": "Large ribosomal subunit protein P1",
  "term_label": "cytosolic large ribosomal subunit",
  "gene_symbol": "RPLP1"
}